{
  "gene_name": "Natural resistance-associated macrophage protein 1",
  "gene": "UniProtKB:P49279",
  "gene_symbol": "SLC11A1",
  "term_id": "GO:0034755",
  "term_label": "iron ion transmembrane transport"
}